glycine-gated chloride channel complex [GO:0016935] (cellular component) Relationships: is a type of chloride channel complex [GO:0034707]; is_a plasma membrane protein complex [GO:0098797] Definition: A protein complex that forms a transmembrane channel through which chloride ions may pass in response to glycine binding to the channel complex or one of its constituent parts. Sources: GOC:mah